{
  "gene": "UniProtKB:P27707",
  "term_label": "cytoplasm",
  "term_id": "GO:0005737",
  "gene_name": "Deoxycytidine kinase",
  "gene_symbol": "DCK"
}